{
  "gene_name": "Thiamine transporter 2",
  "gene": "UniProtKB:Q9BZV2",
  "term_label": "Unknown biological process",
  "gene_symbol": "SLC19A3",
  "term_id": "UNKNOWN:0002"
}